{
  "gene": "UniProtKB:Q6NZY4",
  "gene_symbol": "ZCCHC8",
  "gene_name": "Zinc finger CCHC domain-containing protein 8",
  "term_label": "RNA binding",
  "term_id": "GO:0003723"
}